negative regulation of short-day photoperiodism, flowering [GO:0048577] (biological process) Definition: Any process that stops, prevents or reduces short-day photoperiodism, where the response associated with the photoperiodism is flowering. Flowering is defined by the switch from the vegetative to the reproductive phase. Also known as: down regulation of short-day photoperiodism, flowering, down-regulation of short-day photoperiodism, flowering, downregulation of short-day photoperiodism, flowering, inhibition of short-day photoperiodism, flowering Relationships: is a type of negative regulation of post-embryonic development [GO:0048581]; is a type of negative regulation of response to stimulus [GO:0048585]; is a type of regulation of short-day photoperiodism, flowering [GO:0048587]; negatively regulates GO:0048575 Sources: GOC:jid, GOC:pj, ISBN:0582015952, ISBN:0697037754, ISBN:0709408862